{
  "term_label": "Unknown cellular component",
  "term_id": "UNKNOWN:0003",
  "gene_symbol": "TRBJ2-5",
  "gene": "UniProtKB:A0A0A0MTA4",
  "gene_name": "T cell receptor beta joining 2-5"
}